{
  "gene_name": "Uncharacterized protein",
  "gene_symbol": "A0A2R8Y747",
  "term_label": "insulin receptor binding",
  "term_id": "GO:0005158",
  "gene": "UniProtKB:A0A2R8Y747"
}